L-ascorbate oxidase activity [GO:0008447] (molecular function) Definition: Catalysis of the reaction: 4 L-ascorbate + O2 = 4 monodehydroascorbate + 2 H2O. Sources: RHEA:30243 Also known as: AA oxidase activity, AAO, L-ascorbate:O2 oxidoreductase activity, L-ascorbate:oxygen oxidoreductase activity, L-ascorbic acid oxidase activity, ascorbase activity, ascorbate dehydrogenase activity, ascorbate oxidase activity, ascorbic acid oxidase activity, ascorbic oxidase activity Relationships: is a type of oxidoreductase activity, acting on diphenols and related substances as donors, oxygen as acceptor [GO:0016682]